{
  "gene_symbol": "IGHV3-35",
  "gene": "UniProtKB:A0A0C4DH35",
  "term_id": "GO:0016064",
  "gene_name": "Probable non-functional immunoglobulin heavy variable 3-35",
  "term_label": "immunoglobulin mediated immune response"
}